{
  "term_label": "Unknown cellular component",
  "gene_name": "COMM domain-containing protein 9",
  "gene_symbol": "COMMD9",
  "term_id": "UNKNOWN:0003",
  "gene": "UniProtKB:Q9P000"
}